{
  "gene": "UniProtKB:P24903",
  "term_id": "GO:0016712",
  "term_label": "oxidoreductase activity, acting on paired donors, with incorporation or reduction of molecular oxygen, reduced flavin or flavoprotein as one donor, and incorporation of one atom of oxygen",
  "gene_symbol": "CYP2F1",
  "gene_name": "Cytochrome P450 2F1"
}